{
  "gene_name": "Myotubularin-related protein 5",
  "gene_symbol": "SBF1",
  "term_id": "GO:0005737",
  "gene": "UniProtKB:O95248",
  "term_label": "cytoplasm"
}